triglucosylalkylacylglycerol sulfotransferase activity [GO:0047363] (molecular function) Definition: Catalysis of the reaction: alpha-D-glucosyl-1,6-alpha-D-glucosyl-1,6-alpha-D-glucosyl-1,3-1-O-alkyl-2-O-acylglycerol + 3'-phosphoadenosine 5'-phosphosulfate = 6-sulfo-alpha-D-glucosyl-1,6-alpha-D-glucosyl-1,6-alpha-D-glucosyl-1,3-1-O-alkyl-2-O-acylglycerol + adenosine 3',5'-bisphosphate. Sources: EC:2.8.2.19, MetaCyc:2.8.2.19-RXN Also known as: triglucosylalkylacylglycerol sulphotransferase activity, 3'-phosphoadenylyl-sulfate:triglucosyl-1-O-alkyl-2-O-acylglycerol 6-sulfotransferase activity, triglucosylmonoalkylmonoacyl sulfotransferase activity Relationships: is a type of sulfotransferase activity [GO:0008146]